{
  "gene": "UniProtKB:Q9BUA6",
  "gene_symbol": "MYL10",
  "term_label": "mitochondrion",
  "term_id": "GO:0005739",
  "gene_name": "Myosin regulatory light chain 10"
}